saponin catabolic process [GO:0016136] (biological process) Subtypes: GO:1904462 Also known as: saponin breakdown, saponin catabolism, saponin degradation Definition: The chemical reactions and pathways resulting in the breakdown of saponins, glycosides of plants in which the aglycan (sapogenin) group is a terpene or steroid and the sugar group is a glucose, a galactose, a pentose, a methylpentose or an oligosaccharide. Saponins are powerful surfactant agents and membrane active; they are, hence, toxic to animals on injection. Sources: GOC:go_curators Relationships: is a type of saponin metabolic process [GO:0016134]; is a type of glycoside catabolic process [GO:0016139]